{
  "term_id": "GO:0007399",
  "term_label": "nervous system development",
  "gene": "UniProtKB:P48443",
  "gene_name": "Retinoic acid receptor RXR-gamma",
  "gene_symbol": "RXRG"
}